3,7-dimethylquercitin 4'-O-methyltransferase activity [GO:0030758] (molecular function) Also known as: 3,7-dimethylquercetin 4'-O-methyltransferase activity, 4'-OMT activity, S-adenosyl-L-methionine:3',4',5-trihydroxy-3,7-dimethoxyflavone 4'-O-methyltransferase activity, S-adenosyl-L-methionine:5,3',4'-trihydroxy-3,7-dimethoxyflavone 4'-O-methyltransferase activity, flavonol 4'-O-methyltransferase activity, flavonol 4'-methyltransferase activity Sources: EC:2.1.1.83, RHEA:21832 Relationships: is a type of S-adenosylmethionine-dependent methyltransferase activity [GO:0008757] Definition: Catalysis of the reaction: 3',4',5-trihydroxy-3,7-dimethoxyflavone + S-adenosyl-L-methionine(1+) = 3',5-dihydroxy-3,4',7-trimethoxyflavone + S-adenosyl-L-homocysteine + H+.